phosphoribosylformylglycinamidine cyclo-ligase activity [GO:0004641] (molecular function) Also known as: 2-(formamido)-1-N-(5-phosphoribosyl)acetamidine cyclo-ligase (ADP-forming), 2-(formamido)-N1-(5-phosphoribosyl)acetamidine cyclo-ligase (ADP-forming), 5'-aminoimidazole ribonucleotide synthetase activity, AIR synthase activity, AIR synthetase activity, AIRS activity, phosphoribosyl-aminoimidazole synthetase activity, phosphoribosylaminoimidazole synthetase activity Definition: Catalysis of the reaction: 2-(formamido)-N(1)-(5-phospho-D-ribosyl)acetamidine + ATP = 5-amino-1-(5-phospho-D-ribosyl)imidazole + ADP + 2 H+ + phosphate. Relationships: is a type of cyclo-ligase activity [GO:0016882] Sources: EC:6.3.3.1, RHEA:23032